formate kinase activity [GO:0047900] (molecular function) Sources: EC:2.7.2.6, RHEA:16009 Definition: Catalysis of the reaction: ATP + formate = ADP + formyl phosphate + H+. Relationships: is a type of kinase activity [GO:0016301]; is a type of phosphotransferase activity, carboxyl group as acceptor [GO:0016774] Also known as: ATP:formate phosphotransferase activity